{
  "gene_name": "Small ribosomal subunit protein uS17m",
  "term_label": "Unknown molecular function",
  "gene_symbol": "MRPS17",
  "term_id": "UNKNOWN:0001",
  "gene": "UniProtKB:Q9Y2R5"
}